{
  "gene_name": "Zinc finger Ran-binding domain-containing protein 2",
  "gene": "UniProtKB:O95218",
  "term_label": "lipopolysaccharide binding",
  "term_id": "GO:0001530",
  "gene_symbol": "ZRANB2"
}